{
  "term_id": "GO:0006956",
  "gene_name": "Complement factor H-related protein 5",
  "gene": "UniProtKB:Q9BXR6",
  "term_label": "complement activation",
  "gene_symbol": "CFHR5"
}